{
  "gene_name": "SOSS complex subunit C",
  "term_label": "nucleoplasm",
  "gene": "UniProtKB:Q9NRY2",
  "gene_symbol": "INIP",
  "term_id": "GO:0005654"
}